renal cortex development [GO:0072055] (biological process) Relationships: is_a anatomical structure development [GO:0048856]; is part of kidney development [GO:0001822] Definition: The process whose specific outcome is the progression of the renal cortex over time, from its formation to the mature structure. The renal cortex is the outer region of the kidney. Subtypes: GO:0072214 Sources: GOC:mtg_kidney_jan10